{
  "gene": "UniProtKB:P54652",
  "gene_name": "Heat shock-related 70 kDa protein 2",
  "term_label": "cytoplasm",
  "term_id": "GO:0005737",
  "gene_symbol": "HSPA2"
}